positive regulation of spore-bearing organ development [GO:0075261] (biological process) Subtypes: positive regulation of sorocarp stalk cell differentiation [GO:0031287], positive regulation of conidiophore development [GO:0070795], positive regulation of oogonium development [GO:0075265], GO:0075269, positive regulation of zygosporangium development [GO:0075273], positive regulation of telium development [GO:0075277], positive regulation of uredinium development [GO:0075281], positive regulation of sporangium development [GO:0075311], positive regulation of basidium development [GO:0075315], positive regulation of ascus development [GO:0075319], positive regulation of sporocarp development involved in sexual reproduction [GO:1902060] Relationships: is a type of positive regulation of developmental process [GO:0051094]; is_a positive regulation of multicellular organismal process [GO:0051240]; is a type of regulation of spore-bearing organ development [GO:0075260]; is a type of positive regulation of reproductive process [GO:2000243]; positively regulates spore-bearing structure development [GO:0075259] Sources: GOC:pamgo_curators Definition: Any process that activates, maintains or increases the frequency, rate or extent of spore-bearing organ development, a process in which hyphae grow into special aggregates called fruiting bodies that produce new spores.